{
  "term_label": "regulation of bone mineralization",
  "term_id": "GO:0030500",
  "gene_symbol": "BMP2K",
  "gene": "UniProtKB:Q9NSY1",
  "gene_name": "BMP-2-inducible protein kinase"
}